{
  "gene_name": "Beta-parvin",
  "gene": "UniProtKB:Q9HBI1",
  "gene_symbol": "PARVB",
  "term_id": "GO:0015629",
  "term_label": "actin cytoskeleton"
}